{
  "gene_name": "Calcium-binding protein 7",
  "term_id": "GO:0032588",
  "gene": "UniProtKB:Q86V35",
  "gene_symbol": "CABP7",
  "term_label": "trans-Golgi network membrane"
}